{
  "gene_name": "Alpha-N-acetylgalactosaminide alpha-2,6-sialyltransferase 5",
  "gene_symbol": "ST6GALNAC5",
  "term_label": "oligosaccharide metabolic process",
  "gene": "UniProtKB:Q9BVH7",
  "term_id": "GO:0009311"
}